{
  "term_id": "GO:0007264",
  "term_label": "small GTPase-mediated signal transduction",
  "gene_symbol": "RASL12",
  "gene_name": "Ras-like protein family member 12",
  "gene": "UniProtKB:Q9NYN1"
}